{
  "gene": "UniProtKB:Q8TCT8",
  "gene_symbol": "SPPL2A",
  "gene_name": "Signal peptide peptidase-like 2A",
  "term_id": "GO:0033619",
  "term_label": "membrane protein proteolysis"
}